{
  "gene": "UniProtKB:Q9Y490",
  "term_id": "GO:0005178",
  "gene_symbol": "TLN1",
  "term_label": "integrin binding",
  "gene_name": "Talin-1"
}